{
  "gene": "UniProtKB:Q96IT6",
  "gene_name": "Putative uncharacterized protein ARHGAP5-AS1",
  "gene_symbol": "ARHGAP5-AS1",
  "term_label": "Unknown cellular component",
  "term_id": "UNKNOWN:0003"
}